{
  "gene_symbol": "COL6A5",
  "gene_name": "Collagen alpha-5(VI) chain",
  "term_label": "extracellular matrix organization",
  "term_id": "GO:0030198",
  "gene": "UniProtKB:A8TX70"
}